mitotic spindle astral microtubule end [GO:1905721] (cellular component) Definition: Any microtubule end that is part of a mitotic spindle astral microtubule. Relationships: is a type of GO:1990752; is part of GO:0061673 References: PMID:11007487 Sources: GOC:TermGenie, GO_REF:0000064 Also known as: mitotic spindle astral microtubule tip